{
  "gene_symbol": "CASP4",
  "term_id": "GO:0050729",
  "term_label": "positive regulation of inflammatory response",
  "gene_name": "Caspase-4",
  "gene": "UniProtKB:P49662"
}